{
  "term_label": "chromosome",
  "gene_symbol": "ATM",
  "term_id": "GO:0005694",
  "gene_name": "Serine-protein kinase ATM",
  "gene": "UniProtKB:Q13315"
}